positive regulation of germ tube formation [GO:0075011] (biological process) Sources: GOC:pamgo_curators Definition: Any process that activates, maintains or increases the frequency, rate or extent of germ tube formation on or near host. The host is defined as the larger of the organisms involved in a symbiotic interaction. Also known as: positive regulation of germ tube formation on or near host Relationships: is a type of positive regulation of developmental process [GO:0051094]; is_a regulation of germ tube formation [GO:0075010]; positively regulates germ tube formation [GO:0075009]